{
  "gene": "UniProtKB:P62807",
  "gene_name": "Histone H2B type 1-C_E_F_G_I",
  "term_id": "GO:0019731",
  "term_label": "antibacterial humoral response",
  "gene_symbol": "H2BC10"
}